peptidyl-serine dephosphorylation [GO:0070262] (biological process) Definition: The removal of phosphoric residues from peptidyl-O-phospho-L-serine to form peptidyl-serine. Sources: GOC:bf Relationships: is a type of protein dephosphorylation [GO:0006470]